meiotic DNA repair synthesis involved in reciprocal meiotic recombination [GO:0010778] (biological process) Sources: GOC:dph, GOC:tb Relationships: is a type of meiotic DNA repair synthesis [GO:0000711]; is part of reciprocal meiotic recombination [GO:0007131] Definition: The synthesis of DNA proceeding from the broken 3' single-strand DNA end that uses the homologous intact duplex as the template resulting in meiotic recombination. Meiotic recombination is the cell cycle process in which double strand breaks are formed and repaired through a double Holliday junction intermediate.